{
  "gene_symbol": "CCNJL",
  "gene_name": "Cyclin-J-like protein",
  "gene": "UniProtKB:Q8IV13",
  "term_label": "microtubule organizing center",
  "term_id": "GO:0005815"
}